protein localization to lipid droplet [GO:1990044] (biological process) Relationships: is a type of GO:0033365 References: PMID:22505614 Sources: GOC:sart Also known as: protein localisation to adiposome, protein localisation to lipid body, protein localisation to lipid droplet, protein localisation to lipid particle, protein localization to adiposome, protein localization to lipid body, protein localization to lipid particle Definition: A process in which a protein is transported to, or maintained in, a location on or within a lipid droplet.